fibrillary inclusion [GO:0097408] (cellular component) Definition: Cellular inclusion consisting of circular areas filled with fine slender filaments about 10 nanometers in diameter, delimited by a wall of varying complexity (either a single continuous membrane or a tubular network consisting of a fine filamentous material giving the wall a honeycomb appearance). Fibrillary inclusions are found in the cytoplasm of giant cells of Dieters in the lateral vestibular nucleus of the rat; similar structures have been described in the ventral cochlear nucleus, spinal cord, and substantia nigra. Sources: NIF_Subcellular:sao967812059 Relationships: is a type of inclusion body [GO:0016234]